{
  "gene": "UniProtKB:P51878",
  "term_id": "GO:0043525",
  "gene_symbol": "CASP5",
  "gene_name": "Caspase-5",
  "term_label": "positive regulation of neuron apoptotic process"
}